{
  "gene_name": "Ciliary neurotrophic factor",
  "term_label": "ciliary neurotrophic factor receptor binding",
  "gene_symbol": "CNTF",
  "gene": "UniProtKB:P26441",
  "term_id": "GO:0005127"
}